G protein-coupled chemorepellent receptor activity [GO:0140985] (molecular function) Also known as: G protein chemorepellent receptor activity, G-protein chemorepellent receptor activity, G-protein coupled chemorepellent receptor activity Definition: Combining with a chemorepellent and transmitting the signal across the membrane by activating an associated G-protein; promotes the exchange of GDP for GTP on the alpha subunit of a heterotrimeric G-protein complex. References: PMID:30462573 Relationships: is a type of G protein-coupled receptor activity [GO:0004930]